negative regulation of anoikis [GO:2000811] (biological process) Also known as: negative regulation of detachment induced cell death, negative regulation of suspension induced apoptosis Sources: GOC:obol Definition: Any process that stops, prevents or reduces the frequency, rate or extent of anoikis. Relationships: is a type of negative regulation of apoptotic process [GO:0043066]; is_a regulation of anoikis [GO:2000209]; negatively regulates anoikis [GO:0043276]